{
  "gene_name": "SIN3-HDAC complex-associated factor",
  "gene": "UniProtKB:Q9NP50",
  "term_label": "Unknown molecular function",
  "term_id": "UNKNOWN:0001",
  "gene_symbol": "SINHCAF"
}